{
  "gene_name": "Tetratricopeptide repeat protein 1",
  "gene": "UniProtKB:Q99614",
  "gene_symbol": "TTC1",
  "term_label": "Unknown biological process",
  "term_id": "UNKNOWN:0002"
}